kynurenic acid biosynthetic process [GO:0034276] (biological process) Also known as: 4-hydroxyquinoline-2-carboxylic acid biosynthetic process, kynurenic acid anabolism, kynurenic acid biosynthesis, kynurenic acid synthesis, kynurenic acid formation Sources: GOC:mah Definition: The chemical reactions and pathways resulting in the formation of kynurenic acid, 4-hydroxyquinoline-2-carboxylic acid. Relationships: is a type of GO:0034275; is a type of monocarboxylic acid biosynthetic process [GO:0072330]